{
  "term_id": "GO:0099550",
  "gene_symbol": "CBLN1",
  "term_label": "trans-synaptic signaling, modulating synaptic transmission",
  "gene_name": "Cerebellin-1",
  "gene": "UniProtKB:P23435"
}